{
  "term_id": "GO:0070530",
  "gene": "UniProtKB:Q9Y6K9",
  "gene_name": "NF-kappa-B essential modulator",
  "term_label": "K63-linked polyubiquitin modification-dependent protein binding",
  "gene_symbol": "IKBKG"
}